{
  "term_label": "monoatomic cation channel activity",
  "gene": "UniProtKB:Q9H5I5",
  "gene_name": "Piezo-type mechanosensitive ion channel component 2",
  "term_id": "GO:0005261",
  "gene_symbol": "PIEZO2"
}